regulation of endodeoxyribonuclease activity [GO:0032071] (biological process) Sources: GOC:mah Relationships: is a type of regulation of catalytic activity [GO:0050790]; regulates DNA endonuclease activity [GO:0004520] Definition: Any process that modulates the frequency, rate or extent of endodeoxyribonuclease activity, the hydrolysis of ester linkages within deoxyribonucleic acid by creating internal breaks. Subtypes: positive regulation of endodeoxyribonuclease activity [GO:0032079] Also known as: endodeoxyribonuclease regulator